{
  "term_label": "fatty acid biosynthetic process",
  "gene_name": "3-oxoacyl-[acyl-carrier-protein] reductase",
  "gene": "UniProtKB:Q8N4T8",
  "gene_symbol": "CBR4",
  "term_id": "GO:0006633"
}